{
  "gene_symbol": "OPTN",
  "term_id": "GO:0005737",
  "gene": "UniProtKB:Q96CV9",
  "gene_name": "Optineurin",
  "term_label": "cytoplasm"
}